{
  "term_label": "nucleus",
  "gene_name": "Casein kinase I isoform alpha-like",
  "term_id": "GO:0005634",
  "gene_symbol": "CSNK1A1L",
  "gene": "UniProtKB:Q8N752"
}